cadaverine transport [GO:0015839] (biological process) Relationships: is a type of organic cation transport [GO:0015695]; is_a nitrogen compound transport [GO:0071705] Definition: The directed movement of cadaverine, 1,5-pentanediamine, into, out of or within a cell, or between cells, by means of some agent such as a transporter or pore. Sources: GOC:ai